regulation of protein-containing complex disassembly [GO:0043244] (biological process) Definition: Any process that modulates the frequency, rate or extent of protein complex disassembly, the disaggregation of a protein complex into its constituent components. Sources: GOC:jl Also known as: regulation of protein complex disassembly Relationships: is a type of regulation of cellular component organization [GO:0051128]; regulates protein-containing complex disassembly [GO:0032984] Subtypes: regulation of translational termination [GO:0006449], regulation of termination of DNA-templated transcription [GO:0031554], regulation of SNARE complex disassembly [GO:0035495], negative regulation of protein-containing complex disassembly [GO:0043242], positive regulation of protein-containing complex disassembly [GO:0043243], regulation of myosin II filament disassembly [GO:0043521], GO:0062109, GO:1901096, regulation of protein depolymerization [GO:1901879]